CAG codon-amino acid adaptor activity [GO:0033428] (molecular function) Also known as: glutamine tRNA Note: Note that in the standard genetic code, CAG codes for glutamine. Sources: GOC:mah Relationships: is a type of triplet codon-amino acid adaptor activity [GO:0030533] Definition: A triplet codon-amino acid adaptor activity that recognizes a CAG codon.